{
  "term_id": "UNKNOWN:0002",
  "term_label": "Unknown biological process",
  "gene_symbol": "CMC4",
  "gene_name": "Cx9C motif-containing protein 4",
  "gene": "UniProtKB:P56277"
}